{
  "gene": "UniProtKB:P20648",
  "term_id": "GO:0005391",
  "gene_name": "Potassium-transporting ATPase alpha chain 1",
  "term_label": "P-type sodium:potassium-exchanging transporter activity",
  "gene_symbol": "ATP4A"
}